{
  "term_label": "Unknown biological process",
  "term_id": "UNKNOWN:0002",
  "gene": "UniProtKB:Q2M2E5",
  "gene_name": "Uncharacterized protein C5orf64",
  "gene_symbol": "C5orf64"
}